protein pupylation [GO:0070490] (BP) Relationships: is a type of GO:0018205; is a type of protein modification by small protein conjugation [GO:0032446] Also known as: Pup-protein conjugation, pupylation References: PMID:18980670 Definition: The process in which a Pup protein is conjugated to a target protein via an isopeptide bond between the carboxy-terminus of Pup and the epsilon-amino group of a lysine residue of the target protein.